positive regulation of axonogenesis [GO:0050772] (biological process) Definition: Any process that activates or increases the frequency, rate or extent of axonogenesis. Relationships: is a type of positive regulation of cell projection organization [GO:0031346]; is a type of positive regulation of neurogenesis [GO:0050769]; is a type of regulation of axonogenesis [GO:0050770]; positively regulates axonogenesis [GO:0007409] Subtypes: positive regulation of axon extension [GO:0045773], GO:0048672 Also known as: up regulation of axonogenesis, up-regulation of axonogenesis, upregulation of axonogenesis, activation of axonogenesis, stimulation of axonogenesis Sources: GOC:ai